{
  "gene_symbol": "ZFP14",
  "term_label": "DNA-binding transcription factor activity, RNA polymerase II-specific",
  "gene_name": "Zinc finger protein 14 homolog",
  "term_id": "GO:0000981",
  "gene": "UniProtKB:Q9HCL3"
}